{
  "gene_symbol": "MAEA",
  "gene": "UniProtKB:Q7L5Y9",
  "term_label": "cytoplasm",
  "term_id": "GO:0005737",
  "gene_name": "E3 ubiquitin-protein transferase MAEA"
}